{
  "gene_symbol": "FKBP3",
  "gene": "UniProtKB:Q00688",
  "term_id": "UNKNOWN:0003",
  "gene_name": "Peptidyl-prolyl cis-trans isomerase FKBP3",
  "term_label": "Unknown cellular component"
}